{
  "gene_name": "Selenoprotein V",
  "term_label": "Unknown biological process",
  "term_id": "UNKNOWN:0002",
  "gene_symbol": "SELENOV",
  "gene": "UniProtKB:P59797"
}